{
  "gene_symbol": "YPEL4",
  "gene": "UniProtKB:Q96NS1",
  "term_label": "Unknown biological process",
  "term_id": "UNKNOWN:0002",
  "gene_name": "Protein yippee-like 4"
}